{
  "gene": "UniProtKB:Q92581",
  "gene_name": "Sodium_hydrogen exchanger 6",
  "gene_symbol": "SLC9A6",
  "term_label": "plasma membrane",
  "term_id": "GO:0005886"
}